{
  "term_id": "GO:0005739",
  "gene_symbol": "SUCLA2",
  "gene": "UniProtKB:Q9P2R7",
  "term_label": "mitochondrion",
  "gene_name": "Succinate--CoA ligase [ADP-forming] subunit beta, mitochondrial"
}